{
  "gene_name": "Visual pigment-like receptor peropsin",
  "gene": "UniProtKB:O14718",
  "term_label": "G protein-coupled receptor signaling pathway",
  "gene_symbol": "RRH",
  "term_id": "GO:0007186"
}